{
  "gene_symbol": "PMM1",
  "term_label": "phosphomannomutase activity",
  "term_id": "GO:0004615",
  "gene_name": "Phosphomannomutase 1",
  "gene": "UniProtKB:Q92871"
}